{
  "gene": "UniProtKB:Q2TBC4",
  "term_label": "actin binding",
  "gene_name": "Prickle-like protein 4",
  "gene_symbol": "PRICKLE4",
  "term_id": "GO:0003779"
}